phospholipase A2 inhibitor activity [GO:0019834] (molecular function) Definition: Binds to and stops, prevents or reduces the activity of phospholipase A2. Sources: GOC:ai Relationships: is a type of phospholipase inhibitor activity [GO:0004859]; negatively regulates GO:0004623